{
  "gene_symbol": "SLC27A3",
  "term_label": "endoplasmic reticulum membrane",
  "gene": "UniProtKB:Q5K4L6",
  "term_id": "GO:0005789",
  "gene_name": "Long-chain fatty acid transport protein 3"
}